{
  "gene_name": "ER degradation-enhancing alpha-mannosidase-like protein 1",
  "term_label": "Unknown cellular component",
  "gene": "UniProtKB:Q92611",
  "term_id": "UNKNOWN:0003",
  "gene_symbol": "EDEM1"
}